{
  "term_label": "Unknown biological process",
  "term_id": "UNKNOWN:0002",
  "gene_name": "Grancalcin",
  "gene_symbol": "GCA",
  "gene": "UniProtKB:P28676"
}